{
  "gene_symbol": "LORICRIN",
  "gene_name": "Loricrin",
  "term_label": "cytoplasm",
  "term_id": "GO:0005737",
  "gene": "UniProtKB:P23490"
}